{
  "gene_name": "Zinc finger protein ZIC 4",
  "term_id": "GO:0000981",
  "gene_symbol": "ZIC4",
  "term_label": "DNA-binding transcription factor activity, RNA polymerase II-specific",
  "gene": "UniProtKB:Q8N9L1"
}